phosphatidylcholine-sterol O-acyltransferase activity [GO:0004607] (molecular function) Definition: Catalysis of the reaction: phosphatidylcholine + a sterol = a sterol ester + 1-acylglycerophosphocholine. Regulation: positively regulated by phosphatidylcholine-sterol O-acyltransferase activator activity [GO:0060228] Relationships: is a type of O-acyltransferase activity [GO:0008374] Sources: EC:2.3.1.43 Also known as: LCAT (lecithin-cholesterol acyltransferase), LCAT activity, lecithin--cholesterol acyltransferase activity, lecithin:cholesterol acyltransferase activity, phosphatidylcholine:sterol O-acyltransferase activity, phospholipid--cholesterol acyltransferase activity